{
  "gene_symbol": "GPR75",
  "gene": "UniProtKB:O95800",
  "term_id": "GO:0005886",
  "term_label": "plasma membrane",
  "gene_name": "Probable G-protein coupled receptor 75"
}